{
  "gene_symbol": "RBM3",
  "gene_name": "RNA-binding protein 3",
  "term_id": "GO:0005681",
  "term_label": "spliceosomal complex",
  "gene": "UniProtKB:P98179"
}